DNA amplification [GO:0006277] (biological process) Definition: The process in which the number of copies of a gene is increased in certain cells as extra copies of DNA are made in response to certain signals of cell development or of stress from the environment. Regulation: regulated by regulation of DNA amplification [GO:1904523]; negatively regulated by GO:1904524; positively regulated by GO:1904525 Subtypes: eggshell chorion gene amplification [GO:0007307] Sources: ISBN:0721601464 Relationships: is_a DNA biosynthetic process [GO:0071897]